{
  "gene_name": "T cell receptor alpha variable 12-1",
  "term_id": "UNKNOWN:0002",
  "gene_symbol": "TRAV12-1",
  "gene": "UniProtKB:A0A0B4J245",
  "term_label": "Unknown biological process"
}